DNA-directed RNA polymerase complex [GO:0000428] (cellular component) Definition: A protein complex that possesses DNA-directed RNA polymerase activity. Sources: GOC:krc Relationships: is a type of RNA polymerase complex [GO:0030880] Subtypes: cytosolic DNA-directed RNA polymerase complex [GO:0000345], RNA polymerase IV complex [GO:0000418], GO:0000419, plastid-encoded plastid RNA polymerase complex [GO:0000427], RNA polymerase III complex [GO:0005666], RNA polymerase I complex [GO:0005736], mitochondrial DNA-directed RNA polymerase complex [GO:0034245], GO:0055029